positive regulation of membrane depolarization [GO:1904181] (biological process) References: PMID:20826763 Sources: GOC:TermGenie, GO_REF:0000058 Definition: Any process that activates or increases the frequency, rate or extent of membrane depolarization. Subtypes: positive regulation of mitochondrial depolarization [GO:0051901], positive regulation of membrane depolarization during cardiac muscle cell action potential [GO:1900827], positive regulation of regulation of vascular associated smooth muscle cell membrane depolarization [GO:1904199] Relationships: is a type of GO:0003254; is_a positive regulation of biological process [GO:0048518]; positively regulates GO:0051899 Also known as: up regulation of membrane depolarization, up-regulation of membrane depolarization, upregulation of membrane depolarization, activation of membrane depolarization